{
  "term_id": "GO:0016538",
  "term_label": "cyclin-dependent protein serine/threonine kinase regulator activity",
  "gene_name": "G1_S-specific cyclin-D1",
  "gene": "UniProtKB:P24385",
  "gene_symbol": "CCND1"
}